{
  "term_label": "positive regulation of cytosolic calcium ion concentration",
  "gene_name": "C-C chemokine receptor type 5",
  "term_id": "GO:0007204",
  "gene": "UniProtKB:P51681",
  "gene_symbol": "CCR5"
}